negative regulation of synaptic transmission, dopaminergic [GO:0032227] (biological process) Definition: Any process that stops, prevents, or reduces the frequency, rate or extent of dopaminergic synaptic transmission, the process of communication from a neuron to another neuron across a synapse using the neurotransmitter dopamine. Sources: GOC:mah Also known as: down regulation of synaptic transmission, dopaminergic, down-regulation of synaptic transmission, dopaminergic, downregulation of synaptic transmission, dopaminergic, inhibition of synaptic transmission, dopaminergic Relationships: is a type of regulation of synaptic transmission, dopaminergic [GO:0032225]; is a type of negative regulation of synaptic transmission [GO:0050805]; negatively regulates synaptic transmission, dopaminergic [GO:0001963]